{
  "gene_symbol": "BCORP1",
  "gene": "UniProtKB:Q8N888",
  "term_label": "Unknown molecular function",
  "gene_name": "Putative BCoR-like protein 2",
  "term_id": "UNKNOWN:0001"
}